{
  "term_label": "negative regulation of G2/M transition of mitotic cell cycle",
  "gene_symbol": "PKMYT1",
  "gene_name": "Membrane-associated tyrosine- and threonine-specific cdc2-inhibitory kinase",
  "term_id": "GO:0010972",
  "gene": "UniProtKB:Q99640"
}